{
  "term_label": "Unknown molecular function",
  "gene": "UniProtKB:P04554",
  "gene_name": "Protamine-2",
  "term_id": "UNKNOWN:0001",
  "gene_symbol": "PRM2"
}